{
  "term_label": "Unknown biological process",
  "term_id": "UNKNOWN:0002",
  "gene_name": "Cytochrome P450 27C1",
  "gene": "UniProtKB:Q4G0S4",
  "gene_symbol": "CYP27C1"
}